{
  "term_label": "myelin sheath",
  "term_id": "GO:0043209",
  "gene": "UniProtKB:P07900",
  "gene_symbol": "HSP90AA1",
  "gene_name": "Heat shock protein HSP 90-alpha"
}